{
  "term_id": "GO:0005737",
  "gene": "UniProtKB:Q6IBS0",
  "gene_symbol": "TWF2",
  "gene_name": "Twinfilin-2",
  "term_label": "cytoplasm"
}